{
  "gene_symbol": "ITGA7",
  "gene_name": "Integrin alpha-7",
  "gene": "UniProtKB:Q13683",
  "term_id": "GO:0009986",
  "term_label": "cell surface"
}